{
  "gene": "UniProtKB:Q9GZU1",
  "term_id": "GO:0072345",
  "gene_symbol": "MCOLN1",
  "gene_name": "Mucolipin-1",
  "term_label": "NAADP-sensitive calcium-release channel activity"
}